{
  "term_id": "GO:0031491",
  "term_label": "nucleosome binding",
  "gene_name": "PWWP domain-containing DNA repair factor 3A",
  "gene_symbol": "PWWP3A",
  "gene": "UniProtKB:Q2TAK8"
}